glutathione derivative biosynthetic process [GO:1901687] (biological process) Definition: The chemical reactions and pathways resulting in the formation of glutathione derivative. Sources: GOC:TermGenie, GOC:pr Also known as: glutathione derivative anabolism, glutathione derivative biosynthesis, glutathione derivative formation, glutathione derivative synthesis Relationships: is a type of sulfur compound biosynthetic process [GO:0044272] Subtypes: trypanothione biosynthetic process [GO:0019342]